fractalkine production [GO:0032603] (biological process) Definition: The appearance of fractalkine due to biosynthesis or secretion following a cellular stimulus, resulting in an increase in its intracellular or extracellular levels. References: PMID:12729461 Sources: GOC:mah Relationships: is a type of chemokine production [GO:0032602] Also known as: ABCD-3 production, CX3CL1 production, neurotactin production, fractalkine biosynthetic process, fractalkine metabolic process Regulation: regulated by GO:0032644; negatively regulated by negative regulation of fractalkine production [GO:0032684]; positively regulated by positive regulation of fractalkine production [GO:0032724]